IgE B cell receptor complex [GO:0071744] (cellular component) Note: Note that an IgE immunoglobulin complex has the function of antigen binding if a suitable antigen is available. Also known as: membrane-bound IgE, surface IgE Relationships: is a type of B cell receptor complex [GO:0019815]; is_a GO:0071742 Definition: An IgE immunoglobulin complex that is present in the plasma membrane of B cells and is composed of two identical immunoglobulin heavy chains of the IgE isotype and two identical immunoglobulin light chains and a signaling subunit, a heterodimer of the Ig-alpha and Ig-beta proteins. Sources: GOC:add, ISBN:0781765196